{
  "gene_name": "Golgin subfamily A member 6-like protein 10",
  "gene_symbol": "GOLGA6L10",
  "term_label": "Unknown molecular function",
  "term_id": "UNKNOWN:0001",
  "gene": "UniProtKB:A6NI86"
}